{
  "term_id": "GO:0044183",
  "term_label": "protein folding chaperone",
  "gene": "UniProtKB:P38646",
  "gene_name": "Stress-70 protein, mitochondrial",
  "gene_symbol": "HSPA9"
}